{
  "gene_symbol": "HSP90AA1",
  "term_id": "GO:0034605",
  "gene": "UniProtKB:P07900",
  "term_label": "cellular response to heat",
  "gene_name": "Heat shock protein HSP 90-alpha"
}